{
  "gene": "UniProtKB:Q8IWA0",
  "gene_name": "WD repeat-containing protein 75",
  "gene_symbol": "WDR75",
  "term_id": "GO:0045943",
  "term_label": "positive regulation of transcription by RNA polymerase I"
}